{
  "term_label": "guanyl-nucleotide exchange factor activity",
  "gene_symbol": "RALGPS1",
  "term_id": "GO:0005085",
  "gene_name": "Ras-specific guanine nucleotide-releasing factor RalGPS1",
  "gene": "UniProtKB:Q5JS13"
}